adhesion of symbiont to host via host extracellular matrix [GO:0141018] (biological process) Relationships: is a type of GO:0044406 Also known as: adhesion of symbiont to host extracellular matrix via collagen, adhesion of symbiont to host extracellular matrix via fibronectin, adhesion of symbiont to host extracellular matrix via integrin, adhesion of symbiont to host extracellular matrix via laminin, adhesion of symbiont to host extracellular matrix via vitronectin Definition: The attachment of a symbiont to its host by binding to a component of the host extracellular matrix. The host is defined as the larger of the organisms involved in a symbiotic interaction. References: PMID:15228540, PMID:21270401, PMID:23586629